{
  "term_id": "GO:0061512",
  "gene_symbol": "TULP3",
  "gene": "UniProtKB:O75386",
  "gene_name": "Tubby-related protein 3",
  "term_label": "protein localization to cilium"
}